germ cell proliferation [GO:0036093] (biological process) Definition: The multiplication or reproduction of germ cells, reproductive cells in multicellular organisms, resulting in the expansion of a cell population. Relationships: is a type of GO:0008283; is part of GO:0007276 Regulation: regulated by regulation of germ cell proliferation [GO:1905936]; negatively regulated by GO:1905937; RO_0002213 by positive regulation of germ cell proliferation [GO:1905938] Sources: CL:0000586, GOC:kmv Subtypes: male germ cell proliferation [GO:0002176]